high-affinity oligopeptide transmembrane transporter activity [GO:0015334] (MF) Definition: Enables the transfer of oligopeptide from one side of a membrane to the other. In high-affinity transport the transporter is able to bind the solute even if it is only present at very low concentrations. Oligopeptides are molecules that contain a small number (2 to 20) of amino-acid residues connected by peptide linkages. Sources: GOC:mtg_transport Relationships: is a type of GO:0035673 Also known as: high affinity oligopeptide transporter activity, high-affinity oligopeptide transporter activity